interneuron sorting involved in substrate-independent cerebral cortex tangential migration [GO:0021844] (biological process) Definition: The establishment and response to guidance cues that distribute interneurons to different cerebral cortex structures. References: PMID:12626695 Sources: GOC:cls, GOC:dgh, GOC:dph, GOC:jid, GO_REF:0000021 Relationships: is a type of taxis [GO:0042330]; is part of substrate-independent telencephalic tangential interneuron migration [GO:0021843]